{
  "term_id": "UNKNOWN:0001",
  "gene": "UniProtKB:Q6ZMV7",
  "gene_name": "Protein LEKR1",
  "gene_symbol": "LEKR1",
  "term_label": "Unknown molecular function"
}